CDP catabolic process [GO:0046706] (biological process) Sources: GOC:ai Definition: The chemical reactions and pathways resulting in the breakdown of CDP, cytidine (5'-)diphosphate. Also known as: CDP breakdown, CDP catabolism, CDP degradation Relationships: is a type of pyrimidine ribonucleoside diphosphate catabolic process [GO:0009195]; is a type of GO:0009222; is a type of GO:0046704